regulation of toll-like receptor 1 signaling pathway [GO:0034131] (biological process) Also known as: regulation of TLR1 signaling pathway, regulation of toll-like receptor 1 signalling pathway Definition: Any process that modulates the frequency, rate, or extent of toll-like receptor 1 signaling pathway. References: PMID:16551253, PMID:17328678 Sources: GOC:add Relationships: is a type of regulation of pattern recognition receptor signaling pathway [GO:0062207]; regulates toll-like receptor 1 signaling pathway [GO:0034130] Subtypes: GO:0034132, GO:0034133